{
  "gene_symbol": "SOWAHD",
  "gene_name": "Ankyrin repeat domain-containing protein SOWAHD",
  "term_id": "UNKNOWN:0002",
  "gene": "UniProtKB:A6NJG2",
  "term_label": "Unknown biological process"
}